{
  "gene": "UniProtKB:Q96K80",
  "gene_name": "Zinc finger CCCH domain-containing protein 10",
  "gene_symbol": "ZC3H10",
  "term_id": "UNKNOWN:0003",
  "term_label": "Unknown cellular component"
}